heart formation [GO:0060914] (BP) Definition: The developmental process pertaining to the initial formation of the heart from unspecified parts. This process begins with the specific processes that contribute to the appearance of the heart field and the arrival of cardiac neural crest to the heart region. The process ends when the structural rudiment is recognizable. Also known as: cardiogenesis Relationships: is a type of animal organ formation [GO:0048645]; is part of GO:0003007 Sources: GOC:mtg_heart